border follicle cell migration [GO:0007298] (biological process) Definition: The directed movement of a border cell through the nurse cells to reach the oocyte. An example of this is found in Drosophila melanogaster. References: PMID:10822261 Sources: GOC:mtg_sensu Also known as: border cell migration Relationships: is a type of follicle cell of egg chamber migration [GO:0007297] Regulation: regulated by GO:1903684; negatively regulated by negative regulation of border follicle cell migration [GO:1903687]; positively regulated by positive regulation of border follicle cell migration [GO:1903688]